3-methylbutanal reductase (NADPH) activity [GO:0052675] (molecular function) Definition: Catalysis of the reaction: 3-methylbutanol + NADP+ = 3-methylbutanal + NADPH + H+. 3-methylbutanal is also known as isovaleraldehyde. Sources: RHEA:18525 Also known as: 3-methylbutanal reductase (NADP) activity, 3-methylbutanol:NADP oxidoreductase activity, 3-methylbutyraldehyde reductase (NADP) activity, isoamyl alcohol oxidase (NADP) activity, 3-methylbutanol:NADP+ oxidoreductase activity Relationships: is a type of GO:0008106; is a type of 3-methylbutanal reductase [NAD(P)H] activity [GO:0046568]